microtubule severing ATPase activity [GO:0008568] (molecular function) Definition: Catalysis of the reaction: ATP + H2O = ADP + phosphate. Catalysis of the severing of a microtubule at a specific spot along its length, coupled to the hydrolysis of ATP. Relationships: is a type of polypeptide conformation or assembly isomerase activity [GO:0120544]; is a type of catalytic activity, acting on a protein [GO:0140096]; is a type of GO:0140657; is a type of microtubule destabilizing activity [GO:0170060]; is part of microtubule cytoskeleton organization [GO:0000226] Note: See also the cellular component term 'katanin complex ; GO:0008352'. Also known as: ATP phosphohydrolase (tubulin-dimerizing), microtubule-severing ATPase activity, katanin activity References: PMID:10910766